response to nitroglycerin [GO:1904842] (biological process) Definition: Any process that results in a change in state or activity of a cell or an organism (in terms of movement, secretion, enzyme production, gene expression, etc.) as a result of a nitroglycerin stimulus. Relationships: is a type of GO:1901698; is a type of response to oxygen-containing compound [GO:1901700] References: PMID:25626975 Sources: GOC:TermGenie, GO_REF:0000071 Subtypes: cellular response to nitroglycerin [GO:1904843] Also known as: response to nitroglycerine, response to nitroglycerol, response to trinitroglycerin, response to trinitroglycerol